{
  "term_label": "olfactory receptor activity",
  "gene_symbol": "OR4E1",
  "gene_name": "Olfactory receptor 4E1",
  "gene": "UniProtKB:P0C645",
  "term_id": "GO:0004984"
}